{
  "term_id": "UNKNOWN:0003",
  "term_label": "Unknown cellular component",
  "gene_name": "Putative uncharacterized protein FLJ45840",
  "gene": "UniProtKB:Q6ZS46",
  "gene_symbol": "Q6ZS46"
}